L-methylmalonyl-CoA biosynthetic process [GO:0019680] (biological process) Relationships: is a type of GO:0046491; is a type of acyl-CoA biosynthetic process [GO:0071616] Definition: The chemical reactions and pathways resulting in the formation of L-methylmalonyl-CoA, the L-enantiomer of 2-carboxypropanoyl-CoA. Also known as: L-methylmalonyl-CoA anabolism, L-methylmalonyl-CoA biosynthesis, L-methylmalonyl-CoA formation, L-methylmalonyl-CoA synthesis Sources: GOC:ai, GOC:jsg, GOC:mah